 [go#goslim:pir] Note: PIR GO slim